RNA polymerase III cis-regulatory region sequence-specific DNA binding [GO:0000992] (molecular function) References: PMID:12381659 Sources: GOC:txnOH Relationships: is a type of GO:0000987; is a type of RNA polymerase III transcription regulatory region sequence-specific DNA binding [GO:0001016] Definition: Binding to a specific upstream regulatory DNA sequence (transcription factor recognition sequence or binding site) located in cis relative to the transcription start site (i.e., on the same strand of DNA) of a gene transcribed by RNA polymerase III. The transcribed region might be contain a single gene or a cistron containing multiple genes. Subtypes: RNA polymerase III type 1 promoter sequence-specific DNA binding [GO:0001002], GO:0001003, RNA polymerase III type 3 promoter sequence-specific DNA binding [GO:0001006], RNA polymerase III hybrid type promoter sequence-specific DNA binding [GO:0001039]